negative regulation of lipid droplet fusion [GO:0160078] (biological process) Relationships: is a type of negative regulation of organelle organization [GO:0010639]; negatively regulates lipid droplet fusion [GO:0160077] Definition: Any process that stops, prevents, or reduces the frequency, rate or extent of lipid droplet fusion. References: PMID:36477540